macrophage inflammatory protein-1 alpha production [GO:0071608] (biological process) Relationships: is a type of GO:0032602 Definition: The appearance of macrophage inflammatory protein 1 alpha due to biosynthesis or secretion following a cellular stimulus, resulting in an increase in its intracellular or extracellular levels. Also known as: macrophage inflammatory protein production, CCL3 production, MIP-1a production, chemokine (C-C motif) ligand 3 production Sources: GOC:add, GOC:rv Regulation: regulated by GO:0071640; RO_0002212 by negative regulation of macrophage inflammatory protein 1 alpha production [GO:0071641]; RO_0002213 by positive regulation of macrophage inflammatory protein 1 alpha production [GO:0071642]